{
  "term_id": "GO:0000978",
  "gene": "UniProtKB:Q9HCZ1",
  "gene_name": "Zinc finger protein 334",
  "term_label": "RNA polymerase II cis-regulatory region sequence-specific DNA binding",
  "gene_symbol": "ZNF334"
}